{
  "gene": "UniProtKB:P49908",
  "gene_name": "Selenoprotein P",
  "term_label": "Unknown biological process",
  "gene_symbol": "SELENOP",
  "term_id": "UNKNOWN:0002"
}